{
  "gene_symbol": "TWF1",
  "term_id": "GO:0003785",
  "term_label": "actin monomer binding",
  "gene": "UniProtKB:Q12792",
  "gene_name": "Twinfilin-1"
}